{
  "gene_symbol": "FOLR3",
  "gene_name": "Folate receptor gamma",
  "gene": "UniProtKB:P41439",
  "term_label": "signaling receptor activity",
  "term_id": "GO:0038023"
}